mesenchymal to epithelial transition [GO:0060231] (BP) Also known as: epithelial cell differentiation from mesenchymal cell, mesenchymal-epithelial transition Sources: GOC:ascb_2009, GOC:dph, GOC:tb Subtypes: mesenchymal to epithelial transition involved in metanephros morphogenesis [GO:0003337], mesenchymal to epithelial transition involved in mesonephros morphogenesis [GO:0061261], mesenchymal to epithelial transition involved in renal vesicle formation [GO:0072036] Definition: A transition where a mesenchymal cell establishes apical/basolateral polarity, forms intercellular adhesive junctions, synthesizes basement membrane components and becomes an epithelial cell. Relationships: is a type of GO:0030855